{
  "gene_symbol": "TBX22",
  "gene": "UniProtKB:Q9Y458",
  "term_label": "chromatin",
  "term_id": "GO:0000785",
  "gene_name": "T-box transcription factor TBX22"
}